{
  "gene_symbol": "FRMPD1",
  "term_label": "Unknown biological process",
  "term_id": "UNKNOWN:0002",
  "gene": "UniProtKB:Q5SYB0",
  "gene_name": "FERM and PDZ domain-containing protein 1"
}